{
  "term_label": "microtubule plus-end",
  "gene": "UniProtKB:Q8N3C7",
  "term_id": "GO:0035371",
  "gene_symbol": "CLIP4",
  "gene_name": "CAP-Gly domain-containing linker protein 4"
}